B-1 B cell homeostasis [GO:0001922] (BP) Relationships: is a type of B cell homeostasis [GO:0001782] Sources: GOC:add, ISBN:0781735149 Also known as: B-1 B lymphocyte homeostasis, B-1 B-cell homeostasis, B-1 B-lymphocyte homeostasis Note: Note that this term represents the return of B-1 B cell levels to stable numbers following an immune response, as well as the proliferation and elimination of B-1 B cells in a organism required to maintain stable numbers in the absence of an outside stimulus. Definition: The process of regulating the proliferation and elimination of B cells of the B-1 subset such that the total number of B-1 B cells within a whole or part of an organism is stable over time in the absence of an outside stimulus. B-1 B cells are a distinct subset of B cells characterized as being CD5 positive, found predominantly in the peritoneum, pleural cavities, and spleen, and enriched for self-reactivity.